{
  "gene_symbol": "CBARP",
  "gene_name": "Voltage-dependent calcium channel beta subunit-associated regulatory protein",
  "term_id": "GO:0045955",
  "gene": "UniProtKB:Q8N350",
  "term_label": "negative regulation of calcium ion-dependent exocytosis"
}